{
  "gene_name": "Protein phosphatase inhibitor 2 family member C",
  "term_label": "Unknown cellular component",
  "term_id": "UNKNOWN:0003",
  "gene": "UniProtKB:O14990",
  "gene_symbol": "PPP1R2C"
}